{
  "gene_symbol": "ABHD12B",
  "term_label": "phosphatidylserine catabolic process",
  "term_id": "GO:0006660",
  "gene_name": "Protein ABHD12B",
  "gene": "UniProtKB:Q7Z5M8"
}